response to ribavirin [GO:1901559] (biological process) Sources: GOC:TermGenie Relationships: is a type of response to nitrogen compound [GO:1901698]; is_a response to oxygen-containing compound [GO:1901700] Definition: Any process that results in a change in state or activity of a cell or an organism (in terms of movement, secretion, enzyme production, gene expression, etc.) as a result of a ribavirin stimulus.